{
  "term_label": "organelle transport along microtubule",
  "gene": "UniProtKB:Q969J3",
  "gene_name": "BLOC-1-related complex subunit 5",
  "term_id": "GO:0072384",
  "gene_symbol": "BORCS5"
}